{
  "gene_name": "Tubulin polymerization-promoting protein",
  "term_label": "microtubule polymerization",
  "gene": "UniProtKB:O94811",
  "gene_symbol": "TPPP",
  "term_id": "GO:0046785"
}